{
  "term_id": "GO:0051968",
  "gene_name": "Voltage-dependent calcium channel gamma-5 subunit",
  "gene_symbol": "CACNG5",
  "gene": "UniProtKB:Q9UF02",
  "term_label": "positive regulation of synaptic transmission, glutamatergic"
}